positive regulation of cell cycle phase transition [GO:1901989] (biological process) Also known as: activation of cell cycle transition, positive regulation of cell cycle transition, up regulation of cell cycle phase transition, up regulation of cell cycle transition, up-regulation of cell cycle phase transition, up-regulation of cell cycle transition, upregulation of cell cycle phase transition, upregulation of cell cycle transition, activation of cell cycle phase transition Relationships: is a type of positive regulation of cell cycle process [GO:0090068]; is a type of GO:1901987; positively regulates cell cycle phase transition [GO:0044770] Definition: Any process that activates or increases the frequency, rate or extent of cell cycle phase transition. Subtypes: negative regulation of cell cycle checkpoint [GO:1901977], positive regulation of mitotic cell cycle phase transition [GO:1901992], positive regulation of meiotic cell cycle phase transition [GO:1901995], positive regulation of metaphase/anaphase transition of cell cycle [GO:1902101], GO:1902751, positive regulation of cell cycle G1/S phase transition [GO:1902808] References: PMID:22841721 Sources: GOC:TermGenie, GOC:mtg_cell_cycle